midbrain-hindbrain boundary initiation [GO:0021547] (biological process) Relationships: is a type of regionalization [GO:0003002]; is a type of formation of anatomical boundary [GO:0048859]; is part of neural plate anterior/posterior regionalization [GO:0021999]; is part of midbrain-hindbrain boundary development [GO:0030917] Also known as: MHB biosynthesis, MHB formation, midbrain-hindbrain boundary biosynthesis, midbrain-hindbrain boundary formation, isthmus biosynthesis, isthmus formation References: PMID:15541513 Sources: GOC:cls, GOC:dgh, GOC:dph, GOC:isa_complete, GOC:jid Definition: The regionalization process that gives rise to the midbrain-hindbrain boundary. The midbrain-hindbrain domain of the embryonic brain is comprised of the mesencephalic vesicle and the first rhombencephalic vesicle at early somitogenesis stages. An organizing center at the boundary patterns the midbrain and hindbrain primordia of the neural plate.